myricetin 7-O-methyltransferase activity [GO:0102435] (molecular function) Relationships: is a type of GO:0008168 Definition: Catalysis of the reaction: myricetin + S-adenosyl-L-methionine = 7-O-methylmyricetin + H+ + S-adenosyl-L-homocysteine. Sources: RHEA:74719